{
  "gene": "UniProtKB:Q8IX30",
  "term_id": "GO:0005615",
  "term_label": "extracellular space",
  "gene_name": "Signal peptide, CUB and EGF-like domain-containing protein 3",
  "gene_symbol": "SCUBE3"
}